catecholamine binding [GO:1901338] (molecular function) Sources: GOC:TermGenie Definition: Binding to catecholamine. Subtypes: dopamine binding [GO:0035240], epinephrine binding [GO:0051379], norepinephrine binding [GO:0051380] Relationships: is a type of binding [GO:0005488]